{
  "gene": "UniProtKB:Q9Y366",
  "gene_name": "Intraflagellar transport protein 52 homolog",
  "term_id": "GO:0042073",
  "term_label": "intraciliary transport",
  "gene_symbol": "IFT52"
}